{
  "gene_name": "La-related protein 4",
  "gene_symbol": "LARP4",
  "term_label": "cytosol",
  "gene": "UniProtKB:Q71RC2",
  "term_id": "GO:0005829"
}